{
  "gene_symbol": "SCEL",
  "gene_name": "Sciellin",
  "term_id": "UNKNOWN:0001",
  "gene": "UniProtKB:O95171",
  "term_label": "Unknown molecular function"
}